{
  "gene_symbol": "SLC39A8",
  "gene_name": "Metal cation symporter ZIP8",
  "term_label": "zinc ion import across plasma membrane",
  "term_id": "GO:0071578",
  "gene": "UniProtKB:Q9C0K1"
}